{
  "term_label": "frizzled binding",
  "term_id": "GO:0005109",
  "gene": "UniProtKB:P56706",
  "gene_name": "Protein Wnt-7b",
  "gene_symbol": "WNT7B"
}